{
  "gene_name": "Potassium voltage-gated channel subfamily A member 2",
  "gene": "UniProtKB:P16389",
  "term_id": "GO:0001508",
  "gene_symbol": "KCNA2",
  "term_label": "action potential"
}